{
  "gene_symbol": "KDM4A",
  "term_id": "GO:0032454",
  "term_label": "histone H3K9 demethylase activity",
  "gene_name": "Lysine-specific demethylase 4A",
  "gene": "UniProtKB:O75164"
}